{
  "term_id": "UNKNOWN:0001",
  "gene_name": "Sororin",
  "gene": "UniProtKB:Q96FF9",
  "gene_symbol": "CDCA5",
  "term_label": "Unknown molecular function"
}